{
  "gene_symbol": "NUDT16L1",
  "term_id": "GO:0030515",
  "gene_name": "Tudor-interacting repair regulator protein",
  "gene": "UniProtKB:Q9BRJ7",
  "term_label": "snoRNA binding"
}